trans-4-hydroxy-L-proline catabolic process [GO:0019470] (biological process) Definition: The chemical reactions and pathways resulting in the breakdown of trans-4-hydroxy-L-proline, C5H9NO3, a derivative of the amino acid proline. Sources: GOC:ai Also known as: 4-hydroxyproline breakdown, 4-hydroxyproline catabolism, 4-hydroxyproline degradation Relationships: is a type of modified amino acid catabolic process [GO:0042219]; is a type of L-amino acid catabolic process [GO:0170035]; is a type of non-proteinogenic amino acid catabolic process [GO:0170044]